{
  "gene": "UniProtKB:P35251",
  "gene_symbol": "RFC1",
  "term_id": "GO:0005634",
  "term_label": "nucleus",
  "gene_name": "Replication factor C subunit 1"
}